{
  "gene": "UniProtKB:P53675",
  "term_id": "GO:0032051",
  "gene_symbol": "CLTCL1",
  "term_label": "clathrin light chain binding",
  "gene_name": "Clathrin heavy chain 2"
}